fusogenic activity [GO:0140522] (molecular function) Relationships: is a type of molecular_function [GO:0003674] References: PMID:10332732, PMID:11493675, PMID:12600315, PMID:32100701, PMID:32641474 Definition: The activity of joining two lipid bilayers to form a single membrane. Subtypes: GO:0140523